{
  "gene": "UniProtKB:Q5TIA1",
  "term_id": "GO:0007127",
  "term_label": "meiosis I",
  "gene_name": "Meiosis inhibitor protein 1",
  "gene_symbol": "MEI1"
}